{
  "gene": "UniProtKB:P59047",
  "term_label": "cytosol",
  "gene_symbol": "NLRP5",
  "term_id": "GO:0005829",
  "gene_name": "NACHT, LRR and PYD domains-containing protein 5"
}